{
  "term_id": "GO:0035725",
  "gene": "UniProtKB:P48066",
  "gene_name": "Sodium- and chloride-dependent GABA transporter 3",
  "gene_symbol": "SLC6A11",
  "term_label": "sodium ion transmembrane transport"
}